{
  "gene_name": "Exosome complex component RRP41",
  "gene_symbol": "EXOSC4",
  "gene": "UniProtKB:Q9NPD3",
  "term_label": "nucleolus",
  "term_id": "GO:0005730"
}